nickel incorporation into metallo-sulfur cluster [GO:0018414] (biological process) Subtypes: nickel incorporation into iron-sulfur cluster via tris-L-cysteinyl L-cysteine persulfido L-glutamato L-histidino L-serinyl nickel triiron disulfide trioxide [GO:0018418] Also known as: nickel incorporation into metallo-sulphur cluster Definition: The incorporation of nickel into a metallo-sulfur cluster. Sources: GOC:ai Relationships: is_a metal incorporation into metallo-sulfur cluster [GO:0018282]